negative regulation of base-excision repair [GO:1905052] (biological process) References: PMID:18973764 Sources: GOC:TermGenie, GOC:ah, GO_REF:0000058 Relationships: is a type of negative regulation of DNA repair [GO:0045738]; is a type of GO:1905051; RO_0002212 base-excision repair [GO:0006284] Definition: Any process that stops, prevents or reduces the frequency, rate or extent of base-excision repair. Also known as: down regulation of BER, down regulation of base-excision repair, down-regulation of BER, down-regulation of base-excision repair, downregulation of BER, downregulation of base-excision repair, negative regulation of BER, inhibition of BER, inhibition of base-excision repair